{
  "gene_name": "Transcription factor 7-like 2",
  "gene_symbol": "TCF7L2",
  "term_id": "GO:0060070",
  "gene": "UniProtKB:Q9NQB0",
  "term_label": "canonical Wnt signaling pathway"
}